{
  "term_label": "RNA endonuclease activity",
  "gene": "UniProtKB:Q96J94",
  "gene_name": "Piwi-like protein 1",
  "gene_symbol": "PIWIL1",
  "term_id": "GO:0004521"
}